tRNA (adenine(9)-N1)-methyltransferase activity [GO:0160106] (molecular function) Sources: EC:2.1.1.218 Also known as: tRNA (adenine(9)-N(1))-methyltransferase activity, tRNA m(1)A(9)-methyltransferase, tRNA(m(1)G(9)/m(1)A(9))-methyltransferase Relationships: is a type of tRNA (adenine) methyltransferase activity [GO:0016426] Definition: Catalysis of the reaction: adenosine(9) in tRNA + S-adenosyl-L-methionine = H+ + N(1)-methyladenosine(9) in tRNA + S-adenosyl-L-homocysteine.